{
  "term_label": "cytokine activity",
  "gene_name": "Growth_differentiation factor 7",
  "term_id": "GO:0005125",
  "gene_symbol": "GDF7",
  "gene": "UniProtKB:Q7Z4P5"
}